{
  "term_id": "GO:0034389",
  "term_label": "lipid droplet organization",
  "gene_symbol": "FITM1",
  "gene": "UniProtKB:A5D6W6",
  "gene_name": "Fat storage-inducing transmembrane protein 1"
}